{
  "gene_name": "Cytochrome P450 2A6",
  "gene": "UniProtKB:P11509",
  "term_id": "GO:0005737",
  "gene_symbol": "CYP2A6",
  "term_label": "cytoplasm"
}